{
  "gene_name": "Patatin-like phospholipase domain-containing protein 2",
  "gene": "UniProtKB:Q96AD5",
  "term_label": "lipid homeostasis",
  "gene_symbol": "PNPLA2",
  "term_id": "GO:0055088"
}